{
  "term_label": "transcription coregulator activity",
  "gene_name": "Putative transcription factor SPT20 homolog-like 2",
  "gene": "UniProtKB:P0C7V6",
  "gene_symbol": "SUPT20HL2",
  "term_id": "GO:0003712"
}